trehalose transport [GO:0015771] (biological process) References: PMID:17606922, PMID:20035867 Sources: GOC:ai Definition: The directed movement of trehalose into, out of or within a cell, or between cells, by means of some agent such as a transporter or pore. Trehalose is a disaccharide that consists of two molecules of glucose and is isomeric with sucrose. Relationships: is a type of GO:0015766 Subtypes: trehalose transport in response to water deprivation [GO:0072514]